{
  "term_id": "GO:0005665",
  "gene": "UniProtKB:P61218",
  "gene_symbol": "POLR2F",
  "gene_name": "DNA-directed RNA polymerases I, II, and III subunit RPABC2",
  "term_label": "RNA polymerase II, core complex"
}